{
  "gene_symbol": "FGL2",
  "term_label": "Unknown biological process",
  "gene": "UniProtKB:Q14314",
  "term_id": "UNKNOWN:0002",
  "gene_name": "Fibroleukin"
}